{
  "gene": "UniProtKB:P52742",
  "term_label": "RNA polymerase II cis-regulatory region sequence-specific DNA binding",
  "term_id": "GO:0000978",
  "gene_name": "Zinc finger protein 135",
  "gene_symbol": "ZNF135"
}